immunoglobulin production [GO:0002377] (biological process) Relationships: is a type of production of molecular mediator of immune response [GO:0002440] Also known as: antibody production, immunoglobulin biosynthetic process, immunoglobulin secretion Regulation: regulated by regulation of immunoglobulin production [GO:0002637]; negatively regulated by negative regulation of immunoglobulin production [GO:0002638]; positively regulated by GO:0002639 Note: Note that this term is in the subset of terms that should not be used for direct gene product annotation. Instead, select one of the 'regulation' children terms. Definition: The appearance of immunoglobulin due to biosynthesis or secretion following a cellular stimulus, resulting in an increase in its intracellular or extracellular levels. Sources: GOC:add, ISBN:0781735149 Subtypes: immunoglobulin production involved in immunoglobulin-mediated immune response [GO:0002381]